{
  "term_label": "Unknown molecular function",
  "gene": "UniProtKB:Q9UHA2",
  "term_id": "UNKNOWN:0001",
  "gene_symbol": "SS18L2",
  "gene_name": "SS18-like protein 2"
}